{
  "gene_name": "Rho family-interacting cell polarization regulator 1",
  "gene": "UniProtKB:Q6ZS17",
  "gene_symbol": "RIPOR1",
  "term_label": "cytoplasm",
  "term_id": "GO:0005737"
}